{
  "gene": "UniProtKB:P02461",
  "term_id": "GO:0043588",
  "gene_name": "Collagen alpha-1(III) chain",
  "term_label": "skin development",
  "gene_symbol": "COL3A1"
}